{
  "term_label": "cytoplasm",
  "gene": "UniProtKB:Q96G75",
  "gene_name": "E3 ubiquitin-protein transferase RMND5B",
  "term_id": "GO:0005737",
  "gene_symbol": "RMND5B"
}